{
  "gene_name": "G-protein coupled receptor 37-like 1",
  "gene_symbol": "GPR37L1",
  "gene": "UniProtKB:O60883",
  "term_label": "adenylate cyclase-inhibiting G protein-coupled receptor signaling pathway",
  "term_id": "GO:0007193"
}